{
  "gene": "UniProtKB:O15467",
  "gene_symbol": "CCL16",
  "gene_name": "C-C motif chemokine 16",
  "term_id": "GO:0061844",
  "term_label": "antimicrobial humoral immune response mediated by antimicrobial peptide"
}